mesenchymal cell apoptotic process involved in nephron morphogenesis [GO:1901145] (biological process) Sources: GOC:TermGenie, GOC:mtg_apoptosis Subtypes: mesenchymal cell apoptotic process involved in mesonephric nephron morphogenesis [GO:1901146], mesenchymal cell apoptotic process involved in metanephric nephron morphogenesis [GO:1901147] Definition: Any mesenchymal cell apoptotic process that is involved in nephron morphogenesis. Regulation: regulated by regulation of mesenchymal cell apoptotic process involved in nephron morphogenesis [GO:0072039]; negatively regulated by negative regulation of mesenchymal cell apoptotic process involved in nephron morphogenesis [GO:0072040]; positively regulated by positive regulation of mesenchymal cell apoptotic process involved in nephron morphogenesis [GO:0072041] Relationships: is a type of apoptotic process involved in morphogenesis [GO:0060561]; is a type of mesenchymal cell apoptotic process [GO:0097152]; is part of GO:0072028